vesicle coating [GO:0006901] (biological process) Sources: GOC:jid Definition: A protein coat is added to the vesicle to form the proper shape of the vesicle and to target the vesicle for transport to its destination. Also known as: vesicle coat assembly Relationships: is a type of vesicle organization [GO:0016050]; is part of vesicle budding from membrane [GO:0006900] Subtypes: synaptic vesicle coating [GO:0016183], Golgi transport vesicle coating [GO:0048200], COPII vesicle coating [GO:0048208]